U12 snRNA binding [GO:0030626] (molecular function) Relationships: is a type of GO:0017069 Sources: GOC:jl Definition: Binding to a U12 small nuclear RNA (U12 snRNA).